tabersonine 16-hydroxylase activity [GO:0050594] (molecular function) Relationships: is a type of oxidoreductase activity, acting on paired donors, with incorporation or reduction of molecular oxygen, NAD(P)H as one donor, and incorporation of one atom of oxygen [GO:0016709] Sources: EC:1.14.14.103, RHEA:14133 Also known as: tabersonine,NADPH:oxygen oxidoreductase (16-hydroxylating) Definition: Catalysis of the reaction: H+ + NADPH + O2 + tabersonine = 16-hydroxytabersonine + H2O + NADP+.